{
  "gene": "UniProtKB:P30968",
  "term_label": "plasma membrane",
  "term_id": "GO:0005886",
  "gene_symbol": "GNRHR",
  "gene_name": "Gonadotropin-releasing hormone receptor"
}